{
  "gene": "UniProtKB:Q99967",
  "term_id": "GO:0060972",
  "gene_symbol": "CITED2",
  "gene_name": "Cbp_p300-interacting transactivator 2",
  "term_label": "left/right pattern formation"
}